keratin filament binding [GO:1990254] (molecular function) Relationships: is_a intermediate filament binding [GO:0019215] References: PMID:6170061 Sources: GOC:krc Definition: Binding to a keratin filament, an intermediate filament composed of acidic and basic keratins (types I and II), typically expressed in epithelial cells.